{
  "gene_name": "Serine_threonine-protein kinase SIK3",
  "term_label": "intracellular signal transduction",
  "term_id": "GO:0035556",
  "gene": "UniProtKB:Q9Y2K2",
  "gene_symbol": "SIK3"
}